neural plate axis specification [GO:0021997] (biological process) Relationships: is a type of embryonic axis specification [GO:0000578]; BFO_0000050 neural plate development [GO:0001840]; is part of neural plate pattern specification [GO:0060896] Definition: The pattern specification process in which the axes of the nervous system are established. Sources: GOC:cls, GOC:dgh, GOC:dph, GOC:jid, GO_REF:0000021 Also known as: neural plate axis determination